{
  "gene": "UniProtKB:P54274",
  "gene_symbol": "TERF1",
  "term_id": "GO:0007004",
  "term_label": "telomere maintenance via telomerase",
  "gene_name": "Telomeric repeat-binding factor 1"
}